ascospore wall (1->3)-beta-D-glucan metabolic process [GO:0034409] (BP) Definition: The chemical reactions and pathways involving (1->3)-beta-D-glucans, compounds composed of glucose residues linked by (1->3)-beta-D-glucosidic bonds, found in the walls of ascospores. Relationships: is a type of GO:0034408; is a type of fungal-type cell wall (1->3)-beta-D-glucan metabolic process [GO:0071969] Subtypes: ascospore wall (1->3)-beta-D-glucan biosynthetic process [GO:0034413] Also known as: ascospore wall 1,3-beta-glucan metabolic process, ascospore wall 1,3-beta-D-glucan metabolic process, ascospore wall 1,3-beta-glucan metabolism, ascospore wall beta-1,3 glucan metabolic process, ascospore wall beta-1,3 glucan metabolism Sources: GOC:mah